{
  "gene_name": "Putative golgin subfamily A member 8D",
  "gene": "UniProtKB:Q0D2H9",
  "term_label": "Golgi organization",
  "gene_symbol": "GOLGA8DP",
  "term_id": "GO:0007030"
}